{
  "gene": "UniProtKB:Q9Y2I2",
  "term_id": "GO:0099560",
  "term_label": "synaptic membrane adhesion",
  "gene_symbol": "NTNG1",
  "gene_name": "Netrin-G1"
}